phosphatidylinositol-4,5-bisphosphate phosphatase activity [GO:0106019] (molecular function) Relationships: is a type of phosphatidylinositol bisphosphate phosphatase activity [GO:0034593] Definition: Catalysis of the reaction: 1-phosphatidyl-1D-myo-inositol 4,5-bisphosphate + H2O = 1-phosphatidyl-1D-myo-inositol phosphate + phosphate. Sources: GOC:hjd Subtypes: phosphatidylinositol-4,5-bisphosphate 5-phosphatase activity [GO:0004439], GO:0034597